plant-type cell wall loosening involved in abscission [GO:1902088] (biological process) Relationships: is a type of plant-type cell wall loosening [GO:0009828]; is a type of cell wall modification involved in abscission [GO:0009830] Definition: Any plant-type cell wall loosening that is involved in abscission. Also known as: cellulose and pectin-containing cell wall loosening involved in abscission References: PMID:23479623 Sources: GOC:TermGenie